L-methionine biosynthetic process from homoserine via O-phospho-L-homoserine and cystathionine [GO:0033516] (biological process) Relationships: is a type of GO:0019279 Definition: The chemical reactions and pathways resulting in the formation of L-methionine from other compounds, including homoserine, via the intermediates O-phospho-L-homoserine and cystathionine. Sources: GOC:mah, MetaCyc:PWY-702 Also known as: L-methionine anabolism from homoserine via O-phospho-L-homoserine and cystathionine, L-methionine formation from homoserine via O-phospho-L-homoserine and cystathionine, L-methionine synthesis from homoserine via O-phospho-L-homoserine and cystathionine, methionine biosynthetic process from homoserine via O-phospho-L-homoserine and cystathionine